regulation of iron export across plasma membrane [GO:1904038] (biological process) Definition: Any process that modulates the frequency, rate or extent of export of iron ions from inside of a cell, across the plasma membrane and into the extracellular region. Relationships: is a type of regulation of iron ion transmembrane transport [GO:0034759]; regulates iron ion export across plasma membrane [GO:1903988] References: PMID:15514116 Sources: GOC:BHF, GOC:TermGenie, GOC:kom, GO_REF:0000058 Also known as: regulation of ferrous iron export, regulation of iron(2+) export Subtypes: GO:1904039, GO:1904040